{
  "gene_name": "Paired box protein Pax-7",
  "term_id": "GO:0006357",
  "gene": "UniProtKB:P23759",
  "gene_symbol": "PAX7",
  "term_label": "regulation of transcription by RNA polymerase II"
}